{
  "term_label": "Unknown molecular function",
  "gene": "UniProtKB:P10966",
  "gene_name": "T-cell surface glycoprotein CD8 beta chain",
  "term_id": "UNKNOWN:0001",
  "gene_symbol": "CD8B"
}